alpha-glucuronidase activity [GO:0046559] (molecular function) Relationships: is a type of glucuronidase activity [GO:0046574] Definition: Catalysis of the reaction: an alpha-D-glucuronoside + H2O = an alcohol + D-glucuronate. Sources: EC:3.2.1.139 Also known as: alpha-D-glucosiduronate glucuronohydrolase activity, alpha-glucosiduronase activity